{
  "gene_name": "Grainyhead-like protein 3 homolog",
  "gene_symbol": "GRHL3",
  "term_label": "regulation of transcription by RNA polymerase II",
  "term_id": "GO:0006357",
  "gene": "UniProtKB:Q8TE85"
}